{
  "term_id": "GO:0005776",
  "gene_symbol": "CALCOCO2",
  "gene_name": "Calcium-binding and coiled-coil domain-containing protein 2",
  "term_label": "autophagosome",
  "gene": "UniProtKB:Q13137"
}